{
  "gene_name": "Interleukin-9",
  "gene_symbol": "IL9",
  "gene": "UniProtKB:P15248",
  "term_id": "GO:0005125",
  "term_label": "cytokine activity"
}